{
  "term_label": "prominosome",
  "term_id": "GO:0071914",
  "gene": "UniProtKB:O43490",
  "gene_symbol": "PROM1",
  "gene_name": "Prominin-1"
}